chloroethene reductive dehalogenase activity [GO:0018698] (molecular function) Relationships: is a type of GO:0046992 References: PMID:15294827, PMID:9171062 Sources: RHEA:68004 Also known as: vinyl chloride reductive dehalogenase activity Definition: Catalysis of the reaction: AH2 + chloroethene = A + chloride + ethene + H+.